{
  "gene_symbol": "LGALS2",
  "gene": "UniProtKB:P05162",
  "term_label": "Unknown biological process",
  "term_id": "UNKNOWN:0002",
  "gene_name": "Galectin-2"
}